{
  "gene_name": "Alpha-2A adrenergic receptor",
  "term_id": "GO:0004938",
  "gene_symbol": "ADRA2A",
  "term_label": "alpha2-adrenergic receptor activity",
  "gene": "UniProtKB:P08913"
}